{
  "term_label": "chloride:proton antiporter activity",
  "term_id": "GO:0062158",
  "gene_symbol": "CLCN7",
  "gene": "UniProtKB:P51798",
  "gene_name": "H(+)_Cl(-) exchange transporter 7"
}